early stripe melanocyte differentiation [GO:0050933] (biological process) Relationships: is a type of melanocyte differentiation [GO:0030318] Also known as: early stripe melanocyte cell differentiation, early stripe melanophore differentiation Regulation: regulated by GO:0050939; negatively regulated by negative regulation of early stripe melanocyte differentiation [GO:0050947]; positively regulated by positive regulation of early stripe melanocyte differentiation [GO:0050948] References: PMID:11858836 Definition: The process in which a relatively unspecialized cell acquires the specialized features of an early stripe melanocyte (ESM). In zebrafish, ESMs develop during the first phase (2-3 weeks of development) of the larva to adult transition (2-4 weeks of development).